{
  "gene": "UniProtKB:Q9BX26",
  "term_id": "GO:0000779",
  "gene_symbol": "SYCP2",
  "gene_name": "Synaptonemal complex protein 2",
  "term_label": "condensed chromosome, centromeric region"
}